negative regulation of sporocarp development involved in sexual reproduction [GO:1902059] (biological process) References: PMID:23480775 Sources: GOC:TermGenie, GOC:di Relationships: is a type of negative regulation of spore-bearing organ development [GO:0075262]; is a type of regulation of sporocarp development involved in sexual reproduction [GO:1902058]; negatively regulates sporocarp development involved in sexual reproduction [GO:0000909] Also known as: down regulation of fruiting body development involved in sexual reproduction, down regulation of fruiting body formation involved in sexual reproduction, down-regulation of fruiting body development involved in sexual reproduction, down-regulation of fruiting body formation involved in sexual reproduction, downregulation of fruiting body development involved in sexual reproduction, downregulation of fruiting body formation involved in sexual reproduction, inhibition of fruiting body development involved in sexual reproduction, inhibition of fruiting body formation involved in sexual reproduction, negative regulation of fruiting body development involved in sexual reproduction, negative regulation of fruiting body formation involved in sexual reproduction, down regulation of sporocarp development involved in sexual reproduction, down-regulation of sporocarp development involved in sexual reproduction, downregulation of sporocarp development involved in sexual reproduction, down regulation of ascus development, down regulation of perfect stage fruiting body development, down-regulation of ascus development, down-regulation of perfect stage fruiting body development, downregulation of ascus development, downregulation of perfect stage fruiting body development, inhibition of ascus development, inhibition of perfect stage fruiting body development, inhibition of sporocarp development involved in sexual reproduction, negative regulation of ascus development, negative regulation of perfect stage fruiting body development Subtypes: negative regulation of cleistothecium development [GO:0070797] Definition: Any process that stops, prevents or reduces the frequency, rate or extent of sporocarp development involved in sexual reproduction.